{
  "gene": "UniProtKB:Q92797",
  "gene_name": "Symplekin",
  "term_label": "Unknown molecular function",
  "gene_symbol": "SYMPK",
  "term_id": "UNKNOWN:0001"
}